{
  "gene": "UniProtKB:P10912",
  "term_id": "GO:0070195",
  "gene_name": "Growth hormone receptor",
  "term_label": "growth hormone receptor complex",
  "gene_symbol": "GHR"
}